malate dehydrogenase (decarboxylating) (NAD+) activity [GO:0004471] (molecular function) Relationships: is a type of malic enzyme activity [GO:0004470]; is a type of oxidoreductase activity, acting on the CH-OH group of donors, NAD or NADP as acceptor [GO:0016616] Definition: Catalysis of the reaction: (S)-malate + NAD+ = pyruvate + CO2 + NADH. Also known as: NAD-malic enzyme activity, malate dehydrogenase (oxaloacetate-decarboxylating) activity, 'malic' enzyme, (S)-malate:NAD+ oxidoreductase (decarboxylating), (S)-malate:NAD+ oxidoreductase (oxaloacetate-decarboxylating), NAD-linked malic enzyme, NAD-specific malic enzyme, malate dehydrogenase (decarboxylating) activity Sources: RHEA:12653 Note: For decarboxylation of oxaloacetate (the second substrate listed in EC:1.1.1.38), see 'oxaloacetate decarboxylase activity ; GO:0008948'.